{
  "gene_symbol": "MAFK",
  "gene": "UniProtKB:O60675",
  "term_id": "GO:0006357",
  "gene_name": "Transcription factor MafK",
  "term_label": "regulation of transcription by RNA polymerase II"
}